{
  "term_label": "cell surface",
  "term_id": "GO:0009986",
  "gene": "UniProtKB:O00220",
  "gene_symbol": "TNFRSF10A",
  "gene_name": "Tumor necrosis factor receptor superfamily member 10A"
}